{
  "gene": "UniProtKB:P10451",
  "term_id": "GO:0007155",
  "term_label": "cell adhesion",
  "gene_symbol": "SPP1",
  "gene_name": "Osteopontin"
}